{
  "gene": "UniProtKB:A5PKW4",
  "term_id": "GO:0032587",
  "term_label": "ruffle membrane",
  "gene_symbol": "PSD",
  "gene_name": "PH and SEC7 domain-containing protein 1"
}